{
  "term_id": "GO:0051932",
  "gene_symbol": "GABRD",
  "gene_name": "Gamma-aminobutyric acid receptor subunit delta",
  "gene": "UniProtKB:O14764",
  "term_label": "synaptic transmission, GABAergic"
}